{
  "gene_symbol": "SPINK6",
  "term_label": "extracellular region",
  "gene_name": "Serine protease inhibitor Kazal-type 6",
  "gene": "UniProtKB:Q6UWN8",
  "term_id": "GO:0005576"
}